{
  "gene_symbol": "IGHMBP2",
  "gene_name": "DNA-binding protein SMUBP-2",
  "gene": "UniProtKB:P38935",
  "term_label": "5'-3' DNA helicase activity",
  "term_id": "GO:0043139"
}